{
  "gene_symbol": "Q6ZTI0",
  "gene": "UniProtKB:Q6ZTI0",
  "term_label": "Unknown cellular component",
  "gene_name": "Putative uncharacterized protein FLJ44636",
  "term_id": "UNKNOWN:0003"
}